{
  "gene_name": "Fibulin-7",
  "term_id": "UNKNOWN:0001",
  "gene": "UniProtKB:Q53RD9",
  "term_label": "Unknown molecular function",
  "gene_symbol": "FBLN7"
}